{
  "gene_name": "Glutamate receptor ionotropic, NMDA 3A",
  "term_label": "ionotropic glutamate receptor signaling pathway",
  "gene_symbol": "GRIN3A",
  "gene": "UniProtKB:Q8TCU5",
  "term_id": "GO:0035235"
}